{
  "gene_symbol": "MGMT",
  "term_label": "nucleoplasm",
  "gene": "UniProtKB:P16455",
  "term_id": "GO:0005654",
  "gene_name": "Methylated-DNA--protein-cysteine methyltransferase"
}